positive regulation of gamma-delta T cell differentiation [GO:0045588] (biological process) Definition: Any process that activates or increases the frequency, rate or extent of gamma-delta T cell differentiation. Also known as: positive regulation of gamma-delta T lymphocyte differentiation, positive regulation of gamma-delta T-cell differentiation, positive regulation of gamma-delta T-lymphocyte differentiation, up regulation of gamma-delta T cell differentiation, up-regulation of gamma-delta T cell differentiation, upregulation of gamma-delta T cell differentiation, activation of gamma-delta T cell differentiation, stimulation of gamma-delta T cell differentiation, positive regulation of gamma-delta T cell development Sources: GOC:go_curators Relationships: is a type of positive regulation of T cell differentiation [GO:0045582]; is a type of GO:0045586; is a type of positive regulation of gamma-delta T cell activation [GO:0046645]; positively regulates gamma-delta T cell differentiation [GO:0042492] Note: Note that immunologists typically use the word 'development' to refer to cells of B or T cell lineages undergoing the process that GO describes as 'cell differentiation'.